{
  "gene": "UniProtKB:Q8N8N7",
  "gene_name": "Prostaglandin reductase 2",
  "term_label": "Unknown cellular component",
  "term_id": "UNKNOWN:0003",
  "gene_symbol": "PTGR2"
}